{
  "term_label": "nuclear import signal receptor activity",
  "gene_name": "Importin subunit alpha-5",
  "gene": "UniProtKB:P52294",
  "term_id": "GO:0061608",
  "gene_symbol": "KPNA1"
}